{
  "gene_symbol": "CDC27",
  "gene_name": "Cell division cycle protein 27 homolog",
  "gene": "UniProtKB:P30260",
  "term_label": "cytoplasm",
  "term_id": "GO:0005737"
}